{
  "term_label": "cytoplasm",
  "gene": "UniProtKB:Q6VAB6",
  "gene_symbol": "KSR2",
  "gene_name": "Kinase suppressor of Ras 2",
  "term_id": "GO:0005737"
}